neuroblast fate specification [GO:0014018] (biological process) Relationships: is a type of cell fate specification [GO:0001708]; BFO_0000050 neuroblast fate commitment [GO:0014017] Definition: The process in which a cell becomes capable of differentiating autonomously into a neuroblast in an environment that is neutral with respect to the developmental pathway. Upon specification, the cell fate can be reversed. Sources: GOC:ef, ISBN:0878932585